{
  "gene": "UniProtKB:Q9H497",
  "term_label": "endoplasmic reticulum lumen",
  "term_id": "GO:0005788",
  "gene_name": "Torsin-3A",
  "gene_symbol": "TOR3A"
}